{
  "term_label": "3M complex",
  "term_id": "GO:1990393",
  "gene_symbol": "CUL7",
  "gene": "UniProtKB:Q14999",
  "gene_name": "Cullin-7"
}